{
  "term_id": "GO:0030311",
  "gene_symbol": "B3GNT3",
  "gene_name": "N-acetyllactosaminide beta-1,3-N-acetylglucosaminyltransferase 3",
  "term_label": "poly-N-acetyllactosamine biosynthetic process",
  "gene": "UniProtKB:Q9Y2A9"
}